{
  "gene_name": "Cryptic family protein 1B",
  "gene": "UniProtKB:P0CG36",
  "gene_symbol": "CFC1B",
  "term_label": "cell surface",
  "term_id": "GO:0009986"
}